{
  "gene_symbol": "FGA",
  "gene": "UniProtKB:P02671",
  "term_id": "GO:0005577",
  "term_label": "fibrinogen complex",
  "gene_name": "Fibrinogen alpha chain"
}